gastrulation with mouth forming second [GO:0001702] (biological process) Also known as: deuterostomic gastrulation Definition: A gastrulation process in which the initial invagination becomes the anus and the mouth forms second. Sources: GOC:go_curators, GOC:mtg_sensu Relationships: is a type of gastrulation [GO:0007369]